Cdc73/Paf1 complex [GO:0016593] (cellular component) Definition: A multiprotein complex that associates with RNA polymerase II and general RNA polymerase II transcription factor complexes and may be involved in both transcriptional initiation and elongation. In Saccharomyces the complex contains Paf1p, Cdc73p, Ctr9p, Rtf1p, and Leo1p. Relationships: is a type of transcription elongation factor complex [GO:0008023]; is part of RNA polymerase II, holoenzyme [GO:0016591] References: PMID:11884586 Also known as: Paf1 complex, Paf1p complex